{
  "term_label": "negative regulation of DNA recombination",
  "gene": "UniProtKB:Q02539",
  "gene_name": "Histone H1.1",
  "term_id": "GO:0045910",
  "gene_symbol": "H1-1"
}